{
  "term_id": "GO:0046427",
  "term_label": "positive regulation of receptor signaling pathway via JAK-STAT",
  "gene_symbol": "CSH2",
  "gene": "UniProtKB:P0DML3",
  "gene_name": "Chorionic somatomammotropin hormone 2"
}